{
  "gene": "UniProtKB:Q7RTT9",
  "term_id": "GO:0008504",
  "term_label": "monoamine transmembrane transporter activity",
  "gene_symbol": "SLC29A4",
  "gene_name": "Equilibrative nucleoside transporter 4"
}